medial cortical node [GO:0071341] (cellular component) Definition: A component of the cell division site that contains the mid1, cdr2, wee1, klp8, and blt1 proteins, and is involved in contractile ring localization. Medial cortical node complexes appear as cortical dots in the middle of the cell during interphase, and function to recruit other ring components in early mitosis. Also known as: mid1p medial cortical dot, midsome References: PMID:19474789, PMID:19959363 Sources: GOC:mah, GOC:vw Relationships: is_a GO:0110165; is part of medial cortex [GO:0031097]